{
  "gene": "UniProtKB:P0DMB1",
  "gene_symbol": "PRR23D2",
  "term_id": "UNKNOWN:0001",
  "term_label": "Unknown molecular function",
  "gene_name": "Proline-rich protein 23D2"
}